{
  "gene": "UniProtKB:Q9Y6J6",
  "gene_symbol": "KCNE2",
  "gene_name": "Potassium voltage-gated channel subfamily E member 2",
  "term_id": "GO:0086005",
  "term_label": "ventricular cardiac muscle cell action potential"
}